{
  "gene_name": "CD2 antigen cytoplasmic tail-binding protein 2",
  "gene_symbol": "CD2BP2",
  "term_label": "Unknown molecular function",
  "gene": "UniProtKB:O95400",
  "term_id": "UNKNOWN:0001"
}